{
  "gene": "UniProtKB:Q9Y5S9",
  "term_id": "GO:0003729",
  "term_label": "mRNA binding",
  "gene_symbol": "RBM8A",
  "gene_name": "RNA-binding protein 8A"
}